{
  "gene": "UniProtKB:A6NGU5",
  "term_id": "GO:0036374",
  "gene_symbol": "GGT3P",
  "gene_name": "Putative glutathione hydrolase 3 proenzyme",
  "term_label": "glutathione hydrolase activity"
}